{
  "term_id": "GO:0005737",
  "term_label": "cytoplasm",
  "gene_symbol": "MOCS3",
  "gene_name": "Adenylyltransferase and sulfurtransferase MOCS3",
  "gene": "UniProtKB:O95396"
}